{
  "term_label": "plasma membrane",
  "gene": "UniProtKB:O14795",
  "gene_symbol": "UNC13B",
  "gene_name": "Protein unc-13 homolog B",
  "term_id": "GO:0005886"
}